{
  "term_label": "glycolate biosynthetic process",
  "gene_symbol": "PARK7",
  "gene": "UniProtKB:Q99497",
  "gene_name": "Parkinson disease protein 7",
  "term_id": "GO:0046295"
}